{
  "term_label": "Unknown molecular function",
  "gene": "UniProtKB:Q9GZT3",
  "term_id": "UNKNOWN:0001",
  "gene_symbol": "SLIRP",
  "gene_name": "SRA stem-loop-interacting RNA-binding protein, mitochondrial"
}